{
  "term_id": "GO:0016020",
  "gene_name": "Potassium voltage-gated channel subfamily S member 3",
  "term_label": "membrane",
  "gene": "UniProtKB:Q9BQ31",
  "gene_symbol": "KCNS3"
}